{
  "gene_name": "Phosphatidylinositol 3,4,5-trisphosphate 3-phosphatase TPTE2",
  "term_id": "GO:0016314",
  "gene": "UniProtKB:Q6XPS3",
  "term_label": "phosphatidylinositol-3,4,5-trisphosphate 3-phosphatase activity",
  "gene_symbol": "TPTE2"
}